L-ascorbic acid catabolic process [GO:0019854] (biological process) Also known as: L-ascorbic acid breakdown, L-ascorbic acid catabolism, L-ascorbic acid degradation, ascorbate catabolic process, ascorbate catabolism, vitamin C catabolic process, vitamin C catabolism Sources: GOC:go_curators Relationships: is a type of L-ascorbic acid metabolic process [GO:0019852]; is a type of water-soluble vitamin catabolic process [GO:0042365]; is a type of monosaccharide catabolic process [GO:0046365]; is_a carboxylic acid catabolic process [GO:0046395]; is a type of GO:1901335 Definition: The chemical reactions and pathways resulting in the breakdown of L-ascorbic acid; L-ascorbic acid ionizes to give L-ascorbate, (2R)-2-[(1S)-1,2-dihydroxyethyl]-4-hydroxy-5-oxo-2,5-dihydrofuran-3-olate, which is required as a cofactor in the oxidation of prolyl residues to hydroxyprolyl, and other reactions.